{
  "gene_name": "tRNA N(3)-methylcytidine methyltransferase METTL2A",
  "term_label": "tRNA (cytidine-3-)-methyltransferase activity",
  "term_id": "GO:0052735",
  "gene": "UniProtKB:Q96IZ6",
  "gene_symbol": "METTL2A"
}